{
  "term_id": "GO:0048278",
  "gene_symbol": "STX7",
  "term_label": "vesicle docking",
  "gene": "UniProtKB:O15400",
  "gene_name": "Syntaxin-7"
}